{
  "term_label": "GPI anchor biosynthetic process",
  "gene_name": "Dolichol-phosphate mannosyltransferase subunit 1",
  "gene": "UniProtKB:O60762",
  "term_id": "GO:0006506",
  "gene_symbol": "DPM1"
}